sarcolemma [GO:0042383] (cellular component) Relationships: is a type of plasma membrane [GO:0005886] Definition: The outer membrane of a muscle cell, consisting of the plasma membrane, a covering basement membrane (about 100 nm thick and sometimes common to more than one fiber), and the associated loose network of collagen fibers. Sources: ISBN:0198506732